{
  "gene_name": "Putative exonuclease GOR",
  "term_label": "nucleus",
  "term_id": "GO:0005634",
  "gene_symbol": "REXO1L1P",
  "gene": "UniProtKB:Q8IX06"
}